{
  "gene_symbol": "ZNF722",
  "gene": "UniProtKB:A0A1W2PQL4",
  "gene_name": "Zinc finger protein 722",
  "term_label": "RNA polymerase II cis-regulatory region sequence-specific DNA binding",
  "term_id": "GO:0000978"
}